peptide antibiotic catabolic process [GO:0030652] (biological process) Relationships: is a type of antibiotic catabolic process [GO:0017001]; is a type of peptide catabolic process [GO:0043171]; is a type of GO:0043603 Definition: The chemical reactions and pathways resulting in the breakdown of peptides with antibiotic activity. Subtypes: bacteriocin catabolic process [GO:0046225] Also known as: peptide antibiotic breakdown, peptide antibiotic catabolism, peptide antibiotic degradation Sources: GOC:mah